mesonephric glomerulus vasculature development [GO:0061231] (biological process) Relationships: is a type of glomerulus vasculature development [GO:0072012]; is part of mesonephric glomerulus development [GO:0061224] Definition: The biological process whose specific outcome is the progression of a mesonephric glomerulus vasculature from an initial condition to its mature state. This process begins with the formation of the mesonephric glomerulus vasculature and ends with the mature structure. The mesonephric glomerulus vasculature is composed of the tubule structures that carry blood or lymph in the mesonephric glomerulus. Sources: GOC:mtg_kidney_jan10